{
  "gene_name": "Krueppel-like factor 5",
  "term_id": "GO:0000978",
  "gene": "UniProtKB:Q13887",
  "term_label": "RNA polymerase II cis-regulatory region sequence-specific DNA binding",
  "gene_symbol": "KLF5"
}